{
  "term_id": "GO:0031681",
  "gene_symbol": "GNG8",
  "gene_name": "Guanine nucleotide-binding protein G(I)_G(S)_G(O) subunit gamma-8",
  "term_label": "G-protein beta-subunit binding",
  "gene": "UniProtKB:Q9UK08"
}